regulation of postsynaptic membrane potential [GO:0060078] (biological process) Definition: Any process that modulates the potential difference across a post-synaptic membrane. Sources: GOC:dph, GOC:ef Subtypes: excitatory postsynaptic potential [GO:0060079], inhibitory postsynaptic potential [GO:0060080], hyperpolarization of postsynaptic membrane [GO:0098818], GO:0098819 Also known as: regulation of post-synaptic membrane potential Relationships: is a type of regulation of membrane potential [GO:0042391]